{
  "gene": "UniProtKB:P10632",
  "term_id": "GO:0005737",
  "gene_symbol": "CYP2C8",
  "term_label": "cytoplasm",
  "gene_name": "Cytochrome P450 2C8"
}